{
  "term_label": "plasma membrane",
  "gene_symbol": "CARMIL3",
  "gene": "UniProtKB:Q8ND23",
  "term_id": "GO:0005886",
  "gene_name": "Capping protein, Arp2_3 and myosin-I linker protein 3"
}